{
  "gene_name": "Creatine kinase M-type",
  "gene_symbol": "CKM",
  "gene": "UniProtKB:P06732",
  "term_id": "GO:0005615",
  "term_label": "extracellular space"
}